{
  "term_id": "GO:0006111",
  "gene_symbol": "GNMT",
  "term_label": "regulation of gluconeogenesis",
  "gene_name": "Glycine N-methyltransferase",
  "gene": "UniProtKB:Q14749"
}